{
  "term_label": "cellular response to amino acid stimulus",
  "gene_symbol": "LAMTOR5",
  "gene_name": "Ragulator complex protein LAMTOR5",
  "gene": "UniProtKB:O43504",
  "term_id": "GO:0071230"
}